{
  "gene_name": "Complement factor H",
  "gene_symbol": "CFH",
  "term_label": "complement activation",
  "gene": "UniProtKB:P08603",
  "term_id": "GO:0006956"
}